{
  "gene": "UniProtKB:Q14DG7",
  "term_id": "UNKNOWN:0001",
  "gene_name": "Transmembrane protein 132B",
  "term_label": "Unknown molecular function",
  "gene_symbol": "TMEM132B"
}